stipule development [GO:0010865] (biological process) Definition: The process whose specific outcome is the progression of the stipule over time, from its formation to the mature structure. A stipule is one of (usually) a pair of appendages at the bases of leaves in many broad-leaved angiosperms. Sources: GOC:tb Relationships: is a type of anatomical structure development [GO:0048856]; is part of GO:0048366